{
  "gene": "UniProtKB:Q8N567",
  "term_id": "UNKNOWN:0001",
  "term_label": "Unknown molecular function",
  "gene_symbol": "ZCCHC9",
  "gene_name": "Zinc finger CCHC domain-containing protein 9"
}